{
  "gene_name": "Beclin-2",
  "term_id": "GO:0000407",
  "gene_symbol": "BECN2",
  "gene": "UniProtKB:A8MW95",
  "term_label": "phagophore assembly site"
}